toxic substance binding [GO:0015643] (molecular function) Definition: Binding to a toxic substance, a poisonous substance that causes damage to biological systems. Also known as: antitoxin activity, lipoprotein antitoxin Relationships: is a type of binding [GO:0005488] Sources: GOC:bf, GOC:curators, GOC:jl, GOC:pr